{
  "gene_symbol": "GSK3A",
  "term_label": "negative regulation of TOR signaling",
  "term_id": "GO:0032007",
  "gene": "UniProtKB:P49840",
  "gene_name": "Glycogen synthase kinase-3 alpha"
}